positive regulation of DNA damage response, signal transduction by p53 class mediator [GO:0043517] (biological process) Relationships: is a type of regulation of DNA damage response, signal transduction by p53 class mediator [GO:0043516]; is a type of positive regulation of signal transduction by p53 class mediator [GO:1901798]; positively regulates GO:0030330 Also known as: positive regulation of p53 induced by DNA damage response, up regulation of DNA damage response, signal transduction by p53 class mediator, up-regulation of DNA damage response, signal transduction by p53 class mediator, upregulation of DNA damage response, signal transduction by p53 class mediator, activation of DNA damage response, signal transduction by p53 class mediator, stimulation of DNA damage response, signal transduction by p53 class mediator Sources: GOC:jl Definition: Any process that activates, maintains or increases the rate of the cascade of processes induced by the cell cycle regulator phosphoprotein p53, or an equivalent protein, in response to the detection of DNA damage.